{
  "gene_name": "Disintegrin and metalloproteinase domain-containing protein 2",
  "term_id": "GO:0004222",
  "gene_symbol": "ADAM2",
  "term_label": "metalloendopeptidase activity",
  "gene": "UniProtKB:Q99965"
}